multivesicular body sorting pathway [GO:0071985] (biological process) Subtypes: endosome transport via multivesicular body sorting pathway [GO:0032509] References: PMID:17603537 Sources: GOC:mah Definition: A vesicle-mediated transport process in which transmembrane proteins are ubiquitylated to facilitate their entry into luminal vesicles of multivesicular bodies (MVBs); upon subsequent fusion of MVBs with lysosomes or vacuoles, the cargo proteins are degraded. Relationships: is a type of GO:0016192